1-alkylglycerophosphocholine O-acetyltransferase activity [GO:0047192] (molecular function) Relationships: is a type of O-acetyltransferase activity [GO:0016413] Definition: Catalysis of the reaction: 1-alkyl-sn-glycero-3-phosphocholine + acetyl-CoA = 1-alkyl-2-acetyl-sn-glycero-3-phosphocholine + CoA. Sources: EC:2.3.1.67, MetaCyc:2.3.1.67-RXN Also known as: blood platelet-activating factor acetyltransferase activity, lyso-GPC:acetyl CoA acetyltransferase activity, lyso-platelet activating factor:acetyl-CoA acetyltransferase activity, lyso-platelet-activating factor:acetyl-CoA acetyltransferase activity, lysopaf:acetyl CoA acetyltransferase activity, platelet-activating factor acylhydrolase activity, platelet-activating factor-synthesizing enzyme activity, 1-alkyl-2-lyso-sn-glycero-3-phosphocholine acetyltransferase activity, 1-alkyl-2-lysolecithin acetyltransferase activity, acetyl-CoA:1-alkyl-2-lyso-sn-glycero-3-phosphocholine 2-O-acetyltransferase activity, acetyl-CoA:1-alkyl-sn-glycero-3-phosphocholine 2-O-acetyltransferase activity, acetyl-CoA:lyso-PAF acetyltransferase activity, acyl-CoA:1-alkyl-sn-glycero-3-phosphocholine acyltransferase activity